{
  "term_label": "regulation of transcription by RNA polymerase II",
  "gene_symbol": "CDX1",
  "gene_name": "Homeobox protein CDX-1",
  "gene": "UniProtKB:P47902",
  "term_id": "GO:0006357"
}